{
  "gene": "UniProtKB:P82912",
  "gene_name": "Small ribosomal subunit protein uS11m",
  "gene_symbol": "MRPS11",
  "term_id": "GO:0005763",
  "term_label": "mitochondrial small ribosomal subunit"
}